{
  "term_id": "GO:0008023",
  "gene_name": "RNA polymerase II elongation factor ELL3",
  "term_label": "transcription elongation factor complex",
  "gene_symbol": "ELL3",
  "gene": "UniProtKB:Q9HB65"
}